regulation of phialide development [GO:0070805] (biological process) Sources: GOC:mah Subtypes: negative regulation of phialide development [GO:0070806], GO:0070807 Relationships: is a type of regulation of cell development [GO:0060284]; is a type of regulation of reproductive process [GO:2000241]; regulates phialide development [GO:0070790] Definition: Any process that modulates the frequency, rate or extent of phialide development, a process that leads to the formation of phialides. Phialides are specialized cells that bud from the ends of metulae on the conidiophore tip.